{
  "gene": "UniProtKB:Q8WXI4",
  "term_label": "cytosol",
  "term_id": "GO:0005829",
  "gene_name": "Acyl-coenzyme A thioesterase 11",
  "gene_symbol": "ACOT11"
}